{
  "gene_name": "Adenosine deaminase domain-containing protein 2",
  "gene_symbol": "ADAD2",
  "term_id": "GO:0003726",
  "gene": "UniProtKB:Q8NCV1",
  "term_label": "double-stranded RNA adenosine deaminase activity"
}